{
  "gene_symbol": "GABRD",
  "gene_name": "Gamma-aminobutyric acid receptor subunit delta",
  "gene": "UniProtKB:O14764",
  "term_label": "chloride transmembrane transport",
  "term_id": "GO:1902476"
}